{
  "gene_name": "RNA-binding protein FUS",
  "term_id": "UNKNOWN:0002",
  "term_label": "Unknown biological process",
  "gene": "UniProtKB:P35637",
  "gene_symbol": "FUS"
}